{
  "term_label": "Golgi apparatus",
  "gene_name": "Equilibrative nucleoside transporter 3",
  "gene": "UniProtKB:Q9BZD2",
  "term_id": "GO:0005794",
  "gene_symbol": "SLC29A3"
}